protein import into peroxisome matrix, translocation [GO:0016561] (biological process) References: PMID:11687502 Also known as: peroxisome matrix protein import, translocation, protein translocation during peroxisome matrix protein import, protein translocation during protein import into peroxisome matrix, protein translocation during protein transport into peroxisome matrix, protein transport into peroxisome matrix, translocation, peroxisome receptor translocation Definition: The process in which proteins are moved across the peroxisomal membrane into the matrix. It is likely that the peroxisome targeting sequence receptor remains associated with cargo proteins during translocation. Relationships: is a type of intracellular protein transmembrane transport [GO:0065002]; is part of GO:0016558